{
  "gene_symbol": "NOS3",
  "gene": "UniProtKB:P29474",
  "gene_name": "Nitric oxide synthase 3",
  "term_id": "GO:0005829",
  "term_label": "cytosol"
}